{
  "gene_symbol": "OR10J5",
  "gene": "UniProtKB:Q8NHC4",
  "term_label": "detection of chemical stimulus involved in sensory perception of smell",
  "gene_name": "Olfactory receptor 10J5",
  "term_id": "GO:0050911"
}